{
  "gene": "UniProtKB:O15438",
  "gene_name": "ATP-binding cassette sub-family C member 3",
  "term_label": "ABC-type xenobiotic transporter activity",
  "gene_symbol": "ABCC3",
  "term_id": "GO:0008559"
}